{
  "gene_symbol": "PLPP7",
  "gene_name": "Inactive phospholipid phosphatase 7",
  "term_label": "Unknown biological process",
  "term_id": "UNKNOWN:0002",
  "gene": "UniProtKB:Q8NBV4"
}